{
  "term_label": "3',5'-cyclic-GMP phosphodiesterase activity",
  "term_id": "GO:0047555",
  "gene": "UniProtKB:Q13370",
  "gene_name": "cGMP-inhibited 3',5'-cyclic phosphodiesterase 3B",
  "gene_symbol": "PDE3B"
}